{
  "gene": "UniProtKB:O96018",
  "gene_symbol": "APBA3",
  "gene_name": "Amyloid-beta A4 precursor protein-binding family A member 3",
  "term_id": "GO:0005737",
  "term_label": "cytoplasm"
}